{
  "gene_symbol": "CD8A",
  "term_label": "external side of plasma membrane",
  "gene_name": "T-cell surface glycoprotein CD8 alpha chain",
  "term_id": "GO:0009897",
  "gene": "UniProtKB:P01732"
}